{
  "gene": "UniProtKB:O75459",
  "gene_symbol": "PAGE1",
  "term_id": "UNKNOWN:0002",
  "term_label": "Unknown biological process",
  "gene_name": "P antigen family member 1"
}